{
  "gene_name": "Zinc finger BED domain-containing protein 4",
  "term_id": "UNKNOWN:0003",
  "gene": "UniProtKB:O75132",
  "gene_symbol": "ZBED4",
  "term_label": "Unknown cellular component"
}